{
  "gene_symbol": "NANS",
  "gene": "UniProtKB:Q9NR45",
  "gene_name": "Sialic acid synthase",
  "term_id": "UNKNOWN:0002",
  "term_label": "Unknown biological process"
}